skeletal muscle satellite cell differentiation [GO:0014816] (biological process) Definition: The process in which a relatively unspecialized cell acquires specialized features of a satellite cell. Relationships: is a type of skeletal muscle cell differentiation [GO:0035914] Regulation: negatively regulated by negative regulation of satellite cell differentiation [GO:1902725]; positively regulated by positive regulation of skeletal muscle satellite cell differentiation [GO:1902726] References: PMID:16607119 Sources: GOC:ef, GOC:mtg_muscle